{
  "gene_name": "Eukaryotic initiation factor 4A-II",
  "term_label": "translation initiation factor activity",
  "term_id": "GO:0003743",
  "gene_symbol": "EIF4A2",
  "gene": "UniProtKB:Q14240"
}